{
  "gene_symbol": "CHRDL1",
  "term_label": "negative regulation of BMP signaling pathway",
  "gene": "UniProtKB:Q9BU40",
  "term_id": "GO:0030514",
  "gene_name": "Chordin-like protein 1"
}